{
  "gene": "UniProtKB:Q16706",
  "gene_name": "Alpha-mannosidase 2",
  "gene_symbol": "MAN2A1",
  "term_label": "Golgi membrane",
  "term_id": "GO:0000139"
}